Ski complex [GO:0055087] (cellular component) Definition: A protein complex that regulates RNA degradation by the exosome complex. In Saccharomyces the complex has a heterotetrameric stoichiometry consisting of one copy each of Ski2p and Ski3 and two copies of Ski8p. Relationships: is a type of GO:0032991; is part of cytoplasm [GO:0005737] References: PMID:10744028, PMID:15703439, PMID:16043509, PMID:18042677 Sources: GOC:mcc